{
  "gene_name": "Small nuclear ribonucleoprotein Sm D3",
  "term_id": "GO:0097526",
  "term_label": "spliceosomal tri-snRNP complex",
  "gene": "UniProtKB:P62318",
  "gene_symbol": "SNRPD3"
}